{
  "gene_name": "Acyl-CoA-binding domain-containing protein 7",
  "gene_symbol": "ACBD7",
  "term_label": "fatty-acyl-CoA binding",
  "gene": "UniProtKB:Q8N6N7",
  "term_id": "GO:0000062"
}